{
  "gene": "UniProtKB:Q9Y473",
  "term_id": "UNKNOWN:0003",
  "term_label": "Unknown cellular component",
  "gene_name": "Zinc finger protein 175",
  "gene_symbol": "ZNF175"
}